{
  "term_id": "GO:0005886",
  "gene_name": "Frizzled-3",
  "gene": "UniProtKB:Q9NPG1",
  "gene_symbol": "FZD3",
  "term_label": "plasma membrane"
}